{
  "gene": "UniProtKB:Q53H64",
  "gene_symbol": "ANKRD40CL",
  "term_id": "UNKNOWN:0003",
  "gene_name": "Putative ANKRD40 C-terminal-like protein",
  "term_label": "Unknown cellular component"
}